{
  "term_id": "GO:0005874",
  "gene": "UniProtKB:Q71U36",
  "term_label": "microtubule",
  "gene_symbol": "TUBA1A",
  "gene_name": "Tubulin alpha-1A chain"
}